ent-kaurene oxidase activity [GO:0052615] (molecular function) Definition: Catalysis of the reaction: ent-kaur-16-ene + 3 O2 + 3 reduced [NADPH--hemoprotein reductase] = ent-kaur-16-en-19-oate + 4 H+ + 4 H2O + 3 oxidized [NADPH--hemoprotein reductase]. Relationships: is a type of oxidoreductase activity, acting on paired donors, with incorporation or reduction of molecular oxygen, reduced flavin or flavoprotein as one donor, and incorporation of one atom of oxygen [GO:0016712] Sources: RHEA:32323